chloroplast outer membrane translocon [GO:0010278] (cellular component) Definition: The protein transport machinery of the chloroplast outer membrane that contains at least three components Toc159, Toc75 and Toc34, interacts with precursor proteins which are imported into the chloroplast in a GTP dependant manner. References: PMID:11299338 Relationships: is a type of membrane protein complex [GO:0098796]; is part of GO:0009707